{
  "gene_symbol": "FBXO34",
  "gene": "UniProtKB:Q9NWN3",
  "term_label": "Unknown cellular component",
  "term_id": "UNKNOWN:0003",
  "gene_name": "F-box only protein 34"
}